{
  "term_label": "cytoplasm",
  "gene_name": "Putative GTP-binding protein 6",
  "gene": "UniProtKB:O43824",
  "term_id": "GO:0005737",
  "gene_symbol": "GTPBP6"
}